{
  "term_label": "nucleus",
  "term_id": "GO:0005634",
  "gene_symbol": "XPO1",
  "gene": "UniProtKB:O14980",
  "gene_name": "Exportin-1"
}